{
  "term_label": "bicellular tight junction",
  "gene": "UniProtKB:P56747",
  "term_id": "GO:0005923",
  "gene_symbol": "CLDN6",
  "gene_name": "Claudin-6"
}